{
  "gene_symbol": "GRPEL2",
  "term_label": "protein import into mitochondrial matrix",
  "term_id": "GO:0030150",
  "gene": "UniProtKB:Q8TAA5",
  "gene_name": "GrpE protein homolog 2, mitochondrial"
}